{
  "term_id": "GO:0106333",
  "gene": "UniProtKB:P59047",
  "gene_symbol": "NLRP5",
  "gene_name": "NACHT, LRR and PYD domains-containing protein 5",
  "term_label": "subcortical maternal complex"
}